{
  "term_id": "GO:0008021",
  "term_label": "synaptic vesicle",
  "gene": "UniProtKB:Q8WXE9",
  "gene_name": "Stonin-2",
  "gene_symbol": "STON2"
}